{
  "term_label": "basement membrane assembly",
  "gene": "UniProtKB:Q9HB63",
  "term_id": "GO:0070831",
  "gene_symbol": "NTN4",
  "gene_name": "Netrin-4"
}